{
  "term_id": "UNKNOWN:0003",
  "gene_name": "Leucine-rich repeat-containing protein 18",
  "gene_symbol": "LRRC18",
  "gene": "UniProtKB:Q8N456",
  "term_label": "Unknown cellular component"
}